{
  "term_id": "UNKNOWN:0001",
  "gene_symbol": "CIMAP1A",
  "gene": "UniProtKB:Q96PU9",
  "gene_name": "Outer dense fiber protein 3",
  "term_label": "Unknown molecular function"
}